cuproptosis [GO:0160119] (biological process) Definition: A programmed cell death process that is induced by intracellular copper accumulation. References: PMID:35298263, PMID:35354936 Relationships: is a type of programmed cell death [GO:0012501]